{
  "gene_symbol": "MYBPH",
  "term_id": "GO:0008307",
  "gene": "UniProtKB:Q13203",
  "gene_name": "Myosin-binding protein H",
  "term_label": "structural constituent of muscle"
}